{
  "gene_symbol": "ACP6",
  "gene": "UniProtKB:Q9NPH0",
  "term_id": "GO:2001311",
  "gene_name": "Lysophosphatidic acid phosphatase type 6",
  "term_label": "lysobisphosphatidic acid metabolic process"
}